{
  "gene_name": "Tether containing UBX domain for GLUT4",
  "term_id": "GO:0005634",
  "gene": "UniProtKB:Q9BZE9",
  "term_label": "nucleus",
  "gene_symbol": "ASPSCR1"
}